{
  "gene_symbol": "TMEM30A",
  "gene_name": "Cell cycle control protein 50A",
  "term_label": "phospholipid translocation",
  "term_id": "GO:0045332",
  "gene": "UniProtKB:Q9NV96"
}